{
  "gene": "UniProtKB:P05783",
  "term_label": "intermediate filament cytoskeleton organization",
  "gene_symbol": "KRT18",
  "term_id": "GO:0045104",
  "gene_name": "Keratin, type I cytoskeletal 18"
}